osmosensory signaling via phosphorelay pathway [GO:0007234] (biological process) References: PMID:26787842, PMID:9843501 Also known as: osmolarity sensing via two-component system, osmolarity signaling pathway via two-component system, osmolarity signalling pathway via two-component system, osmosensory signalling pathway via two-component system, signal transduction during osmotic stress via two-component system, osmosensory signaling pathway via two-component system Definition: The series of molecular signals generated in response to osmotic change, as mediated through a phosphorelay system. In S.cerevisiae, the osmosensor is the histidine kinase Sln1. Relationships: is a type of GO:0000160; is a type of osmosensory signaling pathway [GO:0007231]